taste receptor activity [GO:0008527] (molecular function) Definition: Combining with soluble compounds to initiate a change in cell activity. These receptors are responsible for the sense of taste. Sources: GOC:dph Also known as: gustatory receptor Relationships: is a type of transmembrane signaling receptor activity [GO:0004888]; is part of detection of chemical stimulus involved in sensory perception of taste [GO:0050912] Subtypes: GO:0033038, sour taste receptor activity [GO:0033040], sweet taste receptor activity [GO:0033041], GO:0090681, contact chemoreceptor activity [GO:0090684], GO:0170021